{
  "gene_symbol": "NEURL1B",
  "term_label": "ubiquitin protein ligase activity",
  "gene_name": "E3 ubiquitin-protein ligase NEURL1B",
  "gene": "UniProtKB:A8MQ27",
  "term_id": "GO:0061630"
}